{
  "term_label": "fatty acid elongase activity",
  "gene_symbol": "ELOVL3",
  "gene": "UniProtKB:Q9HB03",
  "gene_name": "Elongation of very long chain fatty acids protein 3",
  "term_id": "GO:0009922"
}